{
  "term_id": "GO:0003714",
  "gene_symbol": "RUNX1T1",
  "term_label": "transcription corepressor activity",
  "gene": "UniProtKB:Q06455",
  "gene_name": "Protein CBFA2T1"
}